ecdysteroid biosynthetic process [GO:0045456] (biological process) Regulation: regulated by GO:0007554; RO_0002212 by negative regulation of ecdysteroid biosynthetic process [GO:0045997]; positively regulated by GO:0045998 Subtypes: ecdysone biosynthetic process [GO:0006697] Sources: GOC:go_curators Definition: The chemical reactions and pathways resulting in the formation of ecdysteroids, a group of polyhydroxylated ketosteroids which initiate post-embryonic development. Relationships: is a type of steroid biosynthetic process [GO:0006694]; is a type of ketone biosynthetic process [GO:0042181]; is a type of hormone biosynthetic process [GO:0042446]; is a type of ecdysteroid metabolic process [GO:0045455] Also known as: ecdysteroid anabolism, ecdysteroid biosynthesis, ecdysteroid formation, ecdysteroid synthesis